axon terminus [GO:0043679] (cellular component) Sources: GOC:dph, GOC:jl Also known as: axon terminal, nerve ending, axon terminal specialization Subtypes: calyx of Held [GO:0044305], cone cell pedicle [GO:0044316], vestibular calyx terminal [GO:0099096], Herring body [GO:1990623] Definition: Terminal inflated portion of the axon, containing the specialized apparatus necessary to release neurotransmitters. The axon terminus is considered to be the whole region of thickening and the terminal button is a specialized region of it. Relationships: is a type of neuron projection terminus [GO:0044306]; is_a presynapse [GO:0098793]; is part of distal axon [GO:0150034]